{
  "term_label": "vesicle",
  "gene_symbol": "ACRV1",
  "gene": "UniProtKB:P26436",
  "gene_name": "Acrosomal protein SP-10",
  "term_id": "GO:0031982"
}